carbohydrate phosphorylation [GO:0046835] (biological process) Sources: ISBN:0198506732 Relationships: is a type of GO:0005975; is a type of phosphorylation [GO:0016310] Definition: The process of introducing a phosphate group into a carbohydrate, any organic compound based on the general formula Cx(H2O)y.